{
  "term_id": "UNKNOWN:0001",
  "gene_symbol": "PADI6",
  "term_label": "Unknown molecular function",
  "gene": "UniProtKB:Q6TGC4",
  "gene_name": "Protein-arginine deiminase type-6"
}